{
  "term_id": "GO:0001784",
  "term_label": "phosphotyrosine residue binding",
  "gene_symbol": "GRAP",
  "gene": "UniProtKB:Q13588",
  "gene_name": "GRB2-related adapter protein"
}